{
  "term_id": "GO:0007189",
  "gene_name": "Prostaglandin E2 receptor EP1 subtype",
  "gene_symbol": "PTGER1",
  "term_label": "adenylate cyclase-activating G protein-coupled receptor signaling pathway",
  "gene": "UniProtKB:P34995"
}